{
  "gene": "UniProtKB:P19256",
  "gene_name": "Lymphocyte function-associated antigen 3",
  "term_id": "GO:0009986",
  "gene_symbol": "CD58",
  "term_label": "cell surface"
}